{
  "gene_name": "Endoplasmic reticulum mannosyl-oligosaccharide 1,2-alpha-mannosidase",
  "term_id": "GO:0004571",
  "gene": "UniProtKB:Q9UKM7",
  "term_label": "mannosyl-oligosaccharide 1,2-alpha-mannosidase activity",
  "gene_symbol": "MAN1B1"
}